{
  "gene_symbol": "SH3GL1",
  "term_id": "GO:0030674",
  "term_label": "protein-macromolecule adaptor activity",
  "gene_name": "Endophilin-A2",
  "gene": "UniProtKB:Q99961"
}